{
  "gene": "UniProtKB:Q12913",
  "gene_symbol": "PTPRJ",
  "gene_name": "Receptor-type tyrosine-protein phosphatase eta",
  "term_label": "Unknown cellular component",
  "term_id": "UNKNOWN:0003"
}